{
  "gene": "UniProtKB:Q8TE23",
  "gene_name": "Taste receptor type 1 member 2",
  "term_label": "plasma membrane",
  "term_id": "GO:0005886",
  "gene_symbol": "TAS1R2"
}